{
  "gene": "UniProtKB:O60225",
  "gene_name": "Protein SSX5",
  "term_id": "UNKNOWN:0002",
  "term_label": "Unknown biological process",
  "gene_symbol": "SSX5"
}